{
  "term_id": "GO:0017002",
  "gene_name": "Activin receptor type-2A",
  "gene": "UniProtKB:P27037",
  "term_label": "activin receptor activity",
  "gene_symbol": "ACVR2A"
}